{
  "term_label": "positive regulation of cytosolic calcium ion concentration",
  "term_id": "GO:0007204",
  "gene_symbol": "ADRA1B",
  "gene": "UniProtKB:P35368",
  "gene_name": "Alpha-1B adrenergic receptor"
}